{
  "gene_name": "Interferon alpha-10",
  "gene_symbol": "IFNA10",
  "term_label": "natural killer cell activation involved in immune response",
  "term_id": "GO:0002323",
  "gene": "UniProtKB:P01566"
}